positive regulation of GTPase activity [GO:0043547] (biological process) Relationships: is a type of regulation of GTPase activity [GO:0043087]; is a type of positive regulation of hydrolase activity [GO:0051345]; positively regulates GTPase activity [GO:0003924] Sources: GOC:jl, GOC:mah Definition: Any process that activates or increases the activity of a GTPase. Subtypes: activation of GTPase activity [GO:0090630] Also known as: up regulation of GTPase activity, up-regulation of GTPase activity, upregulation of GTPase activity, activation of GTPase activity, positive regulation of ARF GTPase activity, positive regulation of Cdc42 GTPase activity, positive regulation of Rab GTPase activity, positive regulation of Rac GTPase activity, positive regulation of Ral GTPase activity, positive regulation of Ran GTPase activity, positive regulation of Rap GTPase activity, positive regulation of Ras GTPase activity, positive regulation of Rho GTPase activity, stimulation of ARF GTPase activity, stimulation of Cdc42 GTPase activity, stimulation of GTPase activity, stimulation of Rab GTPase activity, stimulation of Rac GTPase activity, stimulation of Ral GTPase activity, stimulation of Ran GTPase activity, stimulation of Rap GTPase activity, stimulation of Ras GTPase activity, stimulation of Rho GTPase activity, up regulation of ARF GTPase activity, up regulation of Cdc42 GTPase activity, up regulation of Rab GTPase activity, up regulation of Rac GTPase activity, up regulation of Ral GTPase activity, up regulation of Ran GTPase activity, up regulation of Rap GTPase activity, up regulation of Ras GTPase activity, up regulation of Rho GTPase activity, up-regulation of ARF GTPase activity, up-regulation of Cdc42 GTPase activity, up-regulation of Rab GTPase activity, up-regulation of Rac GTPase activity, up-regulation of Ral GTPase activity, up-regulation of Ran GTPase activity, up-regulation of Rap GTPase activity, up-regulation of Ras GTPase activity, up-regulation of Rho GTPase activity, upregulation of ARF GTPase activity, upregulation of Cdc42 GTPase activity, upregulation of Rab GTPase activity, upregulation of Rac GTPase activity, upregulation of Ral GTPase activity, upregulation of Ran GTPase activity, upregulation of Rap GTPase activity, upregulation of Ras GTPase activity, upregulation of Rho GTPase activity